{
  "gene": "UniProtKB:H3BNL8",
  "term_id": "UNKNOWN:0003",
  "gene_symbol": "ARMH2",
  "term_label": "Unknown cellular component",
  "gene_name": "Armadillo-like helical domain-containing protein 2"
}